siderophore metabolic process [GO:0009237] (biological process) Definition: The chemical reactions and pathways involving siderophores, low molecular weight Fe(III)-chelating substances made by aerobic or facultatively anaerobic bacteria, especially when growing under iron deficient conditions. The complexes of Fe(3+)-siderophores have very high stability constants and are taken up by specific transport systems by microorganisms; the subsequent release of iron requires enzymatic action. Subtypes: siderophore biosynthetic process [GO:0019290], vibriobactin metabolic process [GO:0019536], siderophore catabolic process [GO:0046215] Sources: ISBN:0198547684 Relationships: is a type of secondary metabolic process [GO:0019748] Also known as: siderophore metabolism, siderochrome metabolic process, siderochrome metabolism